{
  "gene_name": "Sodium- and chloride-dependent GABA transporter 1",
  "term_id": "GO:0009986",
  "term_label": "cell surface",
  "gene": "UniProtKB:P30531",
  "gene_symbol": "SLC6A1"
}